TRAPPI protein complex [GO:1990070] (cellular component) Relationships: is a type of GO:0030008; is part of endoplasmic reticulum-Golgi intermediate compartment [GO:0005793] References: PMID:20375281, PMID:22669257 Sources: GOC:bhm Also known as: TRAPP core complex Definition: A complex that tethers COPII vesicles at ER-Golgi intermediate compartment. Its role in this part of the vesicular transport may start at the ER exit sites. Binds to a component of the COPII coat. In yeast it includes the following subunits: Bet3 (as homodimer), Bet5, Trs20, Trs23, Trs31, Trs33 which are regarded as the core subunits of all TRAPP complexes in yeast.